Sad1-Kms1 LINC complex [GO:1990612] (cellular component) Definition: A LINC complex implicated in the connection of DNA double strand breaks to the cytoskeleton during DNA double-strand break repair. References: PMID:24943839, PMID:24947240 Sources: GOC:vw Relationships: is_a GO:0034993